{
  "gene_name": "Gem-associated protein 6",
  "term_label": "Unknown molecular function",
  "term_id": "UNKNOWN:0001",
  "gene_symbol": "GEMIN6",
  "gene": "UniProtKB:Q8WXD5"
}